{
  "term_label": "Unknown molecular function",
  "gene_name": "Conserved oligomeric Golgi complex subunit 8",
  "term_id": "UNKNOWN:0001",
  "gene_symbol": "COG8",
  "gene": "UniProtKB:Q96MW5"
}